{
  "gene": "UniProtKB:Q6UXH1",
  "term_id": "GO:0005615",
  "gene_name": "Protein disulfide isomerase CRELD2",
  "term_label": "extracellular space",
  "gene_symbol": "CRELD2"
}